negative regulation of larval salivary gland boundary specification [GO:0045710] (biological process) Relationships: is a type of GO:0045705; is_a GO:0045708; RO_0002212 larval salivary gland boundary specification [GO:0007433] Also known as: down regulation of larval salivary gland determination, down-regulation of larval salivary gland determination, downregulation of larval salivary gland determination, negative regulation of larval salivary gland determination, inhibition of larval salivary gland determination Definition: Any process that stops, prevents, or reduces the frequency, rate or extent of salivary gland determination in a larval organism. Sources: GOC:go_curators, GOC:tb